{
  "term_id": "GO:0000978",
  "gene": "UniProtKB:P48380",
  "gene_name": "Transcription factor RFX3",
  "term_label": "RNA polymerase II cis-regulatory region sequence-specific DNA binding",
  "gene_symbol": "RFX3"
}